{
  "gene": "UniProtKB:Q15388",
  "gene_symbol": "TOMM20",
  "term_id": "GO:0030943",
  "term_label": "mitochondrion targeting sequence binding",
  "gene_name": "Mitochondrial import receptor subunit TOM20 homolog"
}